polyadenylation-dependent ncRNA catabolic process [GO:0043634] (biological process) Definition: The chemical reactions and pathways resulting in the breakdown of a noncoding RNA (ncRNA) molecule, initiated by the enzymatic addition of a sequence of adenylyl residues (polyadenylation) at the 3' end the target ncRNA. Relationships: is a type of polyadenylation-dependent RNA catabolic process [GO:0043633] Subtypes: GO:0035760 Sources: GOC:dgf, GOC:jl, GOC:krc Also known as: poly(A)-dependent ncRNA catabolic process